response to 3,3',5-triiodo-L-thyronine [GO:1905242] (biological process) Definition: Any process that results in a change in state or activity of a cell or an organism (in terms of movement, secretion, enzyme production, gene expression, etc.) as a result of a 3,3',5-triiodo-L-thyronine stimulus. References: PMID:21382270 Sources: GOC:TermGenie, GO_REF:0000071 Also known as: response to Liothyronin, response to Liothyronine, response to Liothyroninum Relationships: is a type of response to amino acid [GO:0043200]; is a type of response to nitrogen compound [GO:1901698]; is_a GO:1901700 Subtypes: cellular response to 3,3',5-triiodo-L-thyronine [GO:1905243]